{
  "term_label": "Unknown molecular function",
  "term_id": "UNKNOWN:0001",
  "gene_name": "Arginine and glutamate-rich protein 1",
  "gene": "UniProtKB:Q9NWB6",
  "gene_symbol": "ARGLU1"
}